alkyl caffeate ester biosynthetic process [GO:0090431] (biological process) Relationships: is_a catechol-containing compound biosynthetic process [GO:0009713]; is a type of cinnamic acid ester biosynthetic process [GO:0009802] Sources: GOC:pz Also known as: alkyl caffeate ester anabolism, alkyl caffeate ester biosynthesis, alkyl caffeate ester formation, alkyl caffeate ester synthesis Definition: The chemical reactions and pathways resulting in the formation of ester derivatives of alkyl caffeate.